peptidyl-isoleucine modification [GO:0018203] (biological process) Relationships: is a type of peptidyl-amino acid modification [GO:0018193] Sources: GOC:go_curators Definition: The modification of peptidyl-isoleucine.